{
  "term_id": "UNKNOWN:0001",
  "gene_name": "Rho guanine nucleotide exchange factor 3",
  "term_label": "Unknown molecular function",
  "gene_symbol": "ARHGEF3",
  "gene": "UniProtKB:Q9NR81"
}